{
  "gene_name": "BEN domain-containing protein 6",
  "gene": "UniProtKB:Q5SZJ8",
  "gene_symbol": "BEND6",
  "term_id": "GO:0005634",
  "term_label": "nucleus"
}